{
  "term_label": "Unknown cellular component",
  "gene": "UniProtKB:O75071",
  "gene_name": "EF-hand calcium-binding domain-containing protein 14",
  "gene_symbol": "EFCAB14",
  "term_id": "UNKNOWN:0003"
}